{
  "term_label": "sensory perception of smell",
  "gene_symbol": "OR5M10",
  "gene": "UniProtKB:Q6IEU7",
  "term_id": "GO:0007608",
  "gene_name": "Olfactory receptor 5M10"
}